{
  "term_label": "DNA-binding transcription factor activity",
  "gene_symbol": "ZNF501",
  "gene": "UniProtKB:Q96CX3",
  "gene_name": "Zinc finger protein 501",
  "term_id": "GO:0003700"
}